{
  "gene_symbol": "DMKN",
  "gene_name": "Dermokine",
  "term_id": "GO:1903575",
  "gene": "UniProtKB:Q6E0U4",
  "term_label": "cornified envelope assembly"
}